{
  "gene_symbol": "PLSCR5",
  "term_id": "GO:0005886",
  "gene_name": "Phospholipid scramblase family member 5",
  "term_label": "plasma membrane",
  "gene": "UniProtKB:A0PG75"
}